{
  "term_id": "GO:0045087",
  "term_label": "innate immune response",
  "gene_name": "WAP four-disulfide core domain protein 12",
  "gene": "UniProtKB:Q8WWY7",
  "gene_symbol": "WFDC12"
}